{
  "gene_symbol": "TCAIM",
  "gene_name": "T-cell activation inhibitor, mitochondrial",
  "gene": "UniProtKB:Q8N3R3",
  "term_id": "UNKNOWN:0002",
  "term_label": "Unknown biological process"
}